{
  "gene_symbol": "GPR37L1",
  "gene_name": "G-protein coupled receptor 37-like 1",
  "term_label": "G protein-coupled peptide receptor activity",
  "gene": "UniProtKB:O60883",
  "term_id": "GO:0008528"
}